{
  "term_label": "lipopolysaccharide binding",
  "gene": "UniProtKB:Q7L0X0",
  "gene_name": "TLR4 interactor with leucine rich repeats",
  "term_id": "GO:0001530",
  "gene_symbol": "TRIL"
}